{
  "gene": "UniProtKB:Q495N2",
  "gene_symbol": "SLC36A3",
  "gene_name": "Proton-coupled amino acid transporter 3",
  "term_id": "GO:0035524",
  "term_label": "proline transmembrane transport"
}